{
  "gene": "UniProtKB:A0A0B4J2D5",
  "gene_symbol": "GATD3B",
  "gene_name": "Putative glutamine amidotransferase-like class 1 domain-containing protein 3B, mitochondrial",
  "term_id": "UNKNOWN:0002",
  "term_label": "Unknown biological process"
}